{
  "term_label": "BMP binding",
  "gene_symbol": "SOSTDC1",
  "term_id": "GO:0036122",
  "gene_name": "Sclerostin domain-containing protein 1",
  "gene": "UniProtKB:Q6X4U4"
}